{
  "term_label": "enzyme regulator activity",
  "gene": "UniProtKB:O94777",
  "gene_name": "Dolichol phosphate-mannose biosynthesis regulatory protein",
  "gene_symbol": "DPM2",
  "term_id": "GO:0030234"
}